{
  "term_label": "regulation of transcription by RNA polymerase II",
  "gene_name": "THAP domain-containing protein 1",
  "gene": "UniProtKB:Q9NVV9",
  "term_id": "GO:0006357",
  "gene_symbol": "THAP1"
}